{
  "gene": "UniProtKB:A6NKF1",
  "term_id": "GO:0005634",
  "term_label": "nucleus",
  "gene_symbol": "SAC3D1",
  "gene_name": "SAC3 domain-containing protein 1"
}